{
  "gene_name": "26S proteasome non-ATPase regulatory subunit 4",
  "gene_symbol": "PSMD4",
  "term_label": "cytosol",
  "gene": "UniProtKB:P55036",
  "term_id": "GO:0005829"
}